{
  "gene_name": "Parathyroid hormone 2 receptor",
  "gene_symbol": "PTH2R",
  "gene": "UniProtKB:P49190",
  "term_label": "plasma membrane",
  "term_id": "GO:0005886"
}